{
  "gene_name": "Nuclear autoantigen Sp-100",
  "gene": "UniProtKB:P23497",
  "gene_symbol": "SP100",
  "term_label": "DNA-binding transcription factor activity, RNA polymerase II-specific",
  "term_id": "GO:0000981"
}